{
  "term_label": "immunoglobulin mediated immune response",
  "gene_name": "Immunoglobulin heavy variable 4-30-4",
  "term_id": "GO:0016064",
  "gene": "UniProtKB:P0DP06",
  "gene_symbol": "IGHV4-30-4"
}